prolactin secreting cell development [GO:0060132] (biological process) Also known as: epsilon-acidophil development, lactotrope development, lactotroph development, lactotropic cell development, mammotrope development, mammotroph development, mammotrophic cell development, mammotropic cell development Relationships: is a type of cell development [GO:0048468]; is part of prolactin secreting cell differentiation [GO:0060127] Definition: The process whose specific outcome is the progression of a prolactin secreting cell over time, from its formation to the mature structure. A prolactin secreting cell is an acidophilic cell of the anterior pituitary that produces prolactin. Sources: GOC:dph